{
  "gene_name": "Substance-K receptor",
  "term_id": "GO:0016497",
  "gene_symbol": "TACR2",
  "gene": "UniProtKB:P21452",
  "term_label": "substance K receptor activity"
}